{
  "gene_name": "Myogenin",
  "gene": "UniProtKB:P15173",
  "term_id": "GO:0035914",
  "term_label": "skeletal muscle cell differentiation",
  "gene_symbol": "MYOG"
}